{
  "term_label": "extracellular space",
  "term_id": "GO:0005615",
  "gene_symbol": "TPSD1",
  "gene": "UniProtKB:Q9BZJ3",
  "gene_name": "Tryptase delta"
}